{
  "gene_name": "Ras association domain-containing protein 2",
  "gene": "UniProtKB:P50749",
  "term_id": "GO:0007165",
  "gene_symbol": "RASSF2",
  "term_label": "signal transduction"
}